extrinsic component of presynaptic active zone membrane [GO:0098891] (cellular component) Sources: GOC:autophagy, GOC:mf Definition: The component of the presynaptic active zone membrane consisting of gene products and protein complexes that are loosely bound to one of its surfaces, but not integrated into the hydrophobic region. Relationships: is a type of extrinsic component of presynaptic membrane [GO:0098888]; is part of presynaptic active zone membrane [GO:0048787]